toxin transmembrane transporter activity [GO:0019534] (molecular function) Definition: Enables the transfer of a toxin from one side of a membrane to the other. A toxin is a poisonous compound (typically a protein) that is produced by cells or organisms and that can cause disease when introduced into the body or tissues of an organism. Sources: ISBN:0198506732 Subtypes: GO:0000269 Relationships: is a type of transmembrane transporter activity [GO:0022857]